{
  "term_id": "UNKNOWN:0001",
  "gene_symbol": "PPFIA3",
  "term_label": "Unknown molecular function",
  "gene": "UniProtKB:O75145",
  "gene_name": "Liprin-alpha-3"
}